plant-type cell wall modification involved in multidimensional cell growth [GO:0009831] (biological process) Definition: The series of events that occur during cell growth that result in chemical or structural changes to existing cell walls of the type composed chiefly of cellulose and pectin. An example of this is found in Arabidopsis thaliana. Also known as: cell wall modification during cell expansion, cellulose and pectin-containing cell wall modification during multidimensional cell growth Relationships: is a type of plant-type cell wall modification [GO:0009827]; is a type of cell wall modification involved in multidimensional cell growth [GO:0042547] Sources: GOC:lr, GOC:mtg_sensu